{
  "gene_symbol": "FRAT2",
  "gene_name": "GSK-3-binding protein FRAT2",
  "term_label": "Unknown molecular function",
  "gene": "UniProtKB:O75474",
  "term_id": "UNKNOWN:0001"
}